proteoglycan sulfotransferase activity [GO:0050698] (molecular function) Subtypes: chondroitin sulfotransferase activity [GO:0034481], heparan sulfate sulfotransferase activity [GO:0034483], GO:0045130, dermatan sulfotransferase activity [GO:0120534] Sources: GOC:ai Also known as: proteoglycan sulphotransferase activity, proteoglycan sulfate transfer Relationships: is a type of sulfotransferase activity [GO:0008146] Definition: Catalysis of the reaction: 3'-phosphoadenosine 5'-phosphosulfate + proteoglycan = adenosine 3',5'-bisphosphate + proteoglycan sulfate. A proteoglycan is a glycoprotein whose carbohydrate units are glycosaminoglycans.